{
  "term_label": "protein targeting to membrane",
  "gene_name": "Palmitoyltransferase ZDHHC23",
  "gene_symbol": "ZDHHC23",
  "term_id": "GO:0006612",
  "gene": "UniProtKB:Q8IYP9"
}